{
  "term_id": "GO:0005737",
  "gene": "UniProtKB:Q9UI30",
  "gene_name": "Multifunctional methyltransferase subunit TRM112-like protein",
  "gene_symbol": "TRMT112",
  "term_label": "cytoplasm"
}